{
  "term_id": "GO:0031594",
  "gene_symbol": "DLG1",
  "gene": "UniProtKB:Q12959",
  "term_label": "neuromuscular junction",
  "gene_name": "Disks large homolog 1"
}